{
  "term_label": "Unknown molecular function",
  "gene_symbol": "ZNF234",
  "term_id": "UNKNOWN:0001",
  "gene": "UniProtKB:Q14588",
  "gene_name": "Zinc finger protein 234"
}